regulation of vein smooth muscle contraction [GO:0062086] (biological process) Definition: Any process that modulates the frequency, rate or extent of vein smooth muscle contraction. References: PMID:8428203 Subtypes: positive regulation of vein smooth muscle contraction [GO:0062087], negative regulation of vein smooth muscle contraction [GO:0062088] Relationships: is a type of regulation of vascular associated smooth muscle contraction [GO:0003056]; regulates vein smooth muscle contraction [GO:0014826]